{
  "gene_name": "Exportin-7",
  "term_label": "protein export from nucleus",
  "gene": "UniProtKB:Q9UIA9",
  "term_id": "GO:0006611",
  "gene_symbol": "XPO7"
}